negative regulation of cyanophore differentiation [GO:0048782] (biological process) Relationships: is a type of GO:0048781; is_a negative regulation of pigment cell differentiation [GO:0050941]; negatively regulates cyanophore differentiation [GO:0048774] Sources: GOC:mh Definition: Any process that stops, prevents, or reduces the frequency, rate or extent of cyanophore differentiation. Also known as: down regulation of cyanophore differentiation, down-regulation of cyanophore differentiation, downregulation of cyanophore differentiation, inhibition of cyanophore differentiation